{
  "term_id": "GO:0031526",
  "gene_name": "Phospholipase B1, membrane-associated",
  "gene": "UniProtKB:Q6P1J6",
  "term_label": "brush border membrane",
  "gene_symbol": "PLB1"
}